{
  "gene": "UniProtKB:O75467",
  "gene_symbol": "ZNF324",
  "term_id": "GO:0005634",
  "gene_name": "Zinc finger protein 324A",
  "term_label": "nucleus"
}